negative regulation of lipid storage [GO:0010888] (biological process) Relationships: is a type of regulation of lipid storage [GO:0010883]; is a type of GO:0048523; is a type of negative regulation of lipid localization [GO:1905953]; negatively regulates lipid storage [GO:0019915] Sources: GOC:BHF, GOC:dph, GOC:tb Subtypes: negative regulation of cholesterol storage [GO:0010887], negative regulation of triglyceride storage [GO:0010891] Definition: Any process that decreases the rate, frequency or extent of lipid storage. Lipid storage is the accumulation and maintenance in cells or tissues of lipids, compounds soluble in organic solvents but insoluble or sparingly soluble in aqueous solvents. Lipid reserves can be accumulated during early developmental stages for mobilization and utilization at later stages of development.